suppression of symbiont entry into host [GO:0052373] (biological process) Relationships: is a type of defense response to symbiont [GO:0140546] Also known as: negative regulation by organism of entry into other organism involved in symbiotic interaction, suppression of symbiont entry into host by host, inhibition by organism of entry into other organism during symbiotic interaction, down regulation by organism of entry into other organism during symbiotic interaction, down-regulation by organism of entry into other organism during symbiotic interaction, downregulation by organism of entry into other organism during symbiotic interaction, negative regulation by organism of entry into other organism during symbiotic interaction Sources: GOC:mtg_pamgo_17jul06 Definition: Any process in which an organism stops, prevents, or reduces the frequency, rate or extent to which it enters into a second organism, where the two organisms are in a symbiotic interaction.